regulation of monoatomic ion transmembrane transport [GO:0034765] (biological process) Definition: Any process that modulates the frequency, rate or extent of the directed movement of ions from one side of a membrane to the other. Subtypes: negative regulation of monoatomic ion transmembrane transport [GO:0034766], GO:0034767, regulation of monoatomic anion transmembrane transport [GO:1903959], regulation of monoatomic cation transmembrane transport [GO:1904062] Relationships: is a type of regulation of transmembrane transport [GO:0034762]; is a type of regulation of monoatomic ion transport [GO:0043269]; regulates monoatomic ion transmembrane transport [GO:0034220] Sources: GOC:mah Also known as: regulation of ion transmembrane transport, regulation of ion membrane transport, regulation of transmembrane ion transport